{
  "gene_symbol": "DNAJC2",
  "gene_name": "DnaJ homolog subfamily C member 2",
  "term_id": "GO:0005829",
  "term_label": "cytosol",
  "gene": "UniProtKB:Q99543"
}